{
  "gene_symbol": "PARP10",
  "gene_name": "Protein mono-ADP-ribosyltransferase PARP10",
  "term_label": "NAD+ poly-ADP-ribosyltransferase activity",
  "term_id": "GO:0003950",
  "gene": "UniProtKB:Q53GL7"
}